phosphopyruvate hydratase activity [GO:0004634] (molecular function) Definition: Catalysis of the reaction: 2-phospho-D-glycerate = phosphoenolpyruvate + H2O. Sources: EC:4.2.1.11, ISBN:0198506732 Also known as: 2-phospho-D-glycerate-hydrolase activity, nervous-system specific enolase, 14-3-2-protein, 2-phospho-D-glycerate hydro-lyase (phosphoenolpyruvate-forming), 2-phospho-D-glycerate hydro-lyase activity, 2-phosphoglycerate dehydratase activity, 2-phosphoglycerate enolase activity, 2-phosphoglyceric dehydratase activity, enolase activity, gamma-enolase activity, phosphoenolpyruvate hydratase activity Relationships: is a type of hydro-lyase activity [GO:0016836]